{
  "term_label": "DNA-binding transcription factor activity, RNA polymerase II-specific",
  "gene_symbol": "ZNF696",
  "gene_name": "Zinc finger protein 696",
  "term_id": "GO:0000981",
  "gene": "UniProtKB:Q9H7X3"
}